{
  "gene": "UniProtKB:Q03701",
  "term_label": "Unknown biological process",
  "gene_symbol": "CEBPZ",
  "term_id": "UNKNOWN:0002",
  "gene_name": "CCAAT_enhancer-binding protein zeta"
}